{
  "gene": "UniProtKB:Q9NUE0",
  "term_id": "GO:0019706",
  "term_label": "protein-cysteine S-palmitoyltransferase activity",
  "gene_symbol": "ZDHHC18",
  "gene_name": "Palmitoyltransferase ZDHHC18"
}